{
  "term_id": "GO:0006952",
  "gene_name": "Dual oxidase 1",
  "gene": "UniProtKB:Q9NRD9",
  "gene_symbol": "DUOX1",
  "term_label": "defense response"
}